cellular response to cell-matrix adhesion [GO:0071460] (biological process) Definition: Any process that results in a change in state or activity of a cell (in terms of movement, secretion, enzyme production, gene expression, etc.) as a result of cell-matrix adhesion. References: PMID:11425869 Sources: GOC:sl Relationships: is a type of cellular response to stimulus [GO:0051716]